{
  "gene": "UniProtKB:P61326",
  "gene_name": "Protein mago nashi homolog",
  "term_label": "Unknown molecular function",
  "term_id": "UNKNOWN:0001",
  "gene_symbol": "MAGOH"
}